{
  "term_id": "GO:0043048",
  "gene_symbol": "DOLK",
  "gene_name": "Dolichol kinase",
  "gene": "UniProtKB:Q9UPQ8",
  "term_label": "dolichyl monophosphate biosynthetic process"
}